mitotic G2/M transition checkpoint [GO:0044818] (biological process) Definition: A cell cycle checkpoint that detects and negatively regulates progression from G2 to M phase as part of a mitotic cell cycle. Subtypes: GO:0007095, GO:0033314 Relationships: is_a mitotic cell cycle checkpoint signaling [GO:0007093]; is a type of negative regulation of G2/M transition of mitotic cell cycle [GO:0010972] Sources: GOC:mtg_cell_cycle